{
  "gene_symbol": "LINC00469",
  "gene_name": "Putative uncharacterized protein encoded by LINC00469",
  "term_label": "Unknown cellular component",
  "gene": "UniProtKB:Q8N7U9",
  "term_id": "UNKNOWN:0003"
}